{
  "gene_name": "Serine_threonine-protein kinase Nek2",
  "term_id": "GO:0000086",
  "term_label": "G2/M transition of mitotic cell cycle",
  "gene_symbol": "NEK2",
  "gene": "UniProtKB:P51955"
}